chemoattraction of serotonergic neuron axon [GO:0036517] (biological process) Definition: The process in which a serotonergic neuron growth cone is directed to a specific target site in response to an attractive chemical signal. References: PMID:21106844 Sources: CL:0000850, GOC:PARL, GOC:bf Also known as: chemoattraction of 5-HT axon, chemoattraction of serotonergic axon Relationships: is_a chemoattraction of axon [GO:0061642]; is part of GO:0036515